{
  "term_id": "UNKNOWN:0001",
  "gene": "UniProtKB:Q9H939",
  "gene_symbol": "PSTPIP2",
  "gene_name": "Proline-serine-threonine phosphatase-interacting protein 2",
  "term_label": "Unknown molecular function"
}